{
  "term_label": "Unknown biological process",
  "gene_symbol": "MMD2",
  "gene": "UniProtKB:Q8IY49",
  "gene_name": "Monocyte to macrophage differentiation factor 2",
  "term_id": "UNKNOWN:0002"
}